antifungal innate immune response [GO:0061760] (biological process) Definition: An defense response against a fungus mediated through an innate immune response. An innate immune response is mediated by germline encoded components that directly recognize components of potential pathogens. Relationships: is a type of innate immune response [GO:0045087]; is a type of defense response to fungus [GO:0050832] Regulation: regulated by GO:1905034; negatively regulated by negative regulation of antifungal innate immune response [GO:1905035]; positively regulated by positive regulation of antifungal innate immune response [GO:1905036] References: PMID:22470487 Sources: GOC:dph